{
  "term_id": "GO:0016446",
  "gene_symbol": "MLH1",
  "gene": "UniProtKB:P40692",
  "term_label": "somatic hypermutation of immunoglobulin genes",
  "gene_name": "DNA mismatch repair protein Mlh1"
}